mitotic DNA replication checkpoint signaling [GO:0033314] (biological process) Definition: A signal transduction process that contributes to a mitotic DNA replication checkpoint. Also known as: S-phase checkpoint, S-M DNA replication checkpoint, S-M checkpoint, mitotic DNA replication checkpoint, mitotic cell cycle DNA replication checkpoint, signal transduction involved in S-M checkpoint, signal transduction involved in mitotic DNA replication checkpoint, signal transduction involved in mitotic G2/M transition decatenation checkpoint Sources: GOC:mtg_cell_cycle Relationships: is a type of GO:0000076; is a type of mitotic DNA integrity checkpoint signaling [GO:0044774]; is a type of mitotic G2/M transition checkpoint [GO:0044818]